{
  "gene_symbol": "CLDN34",
  "term_label": "bicellular tight junction",
  "gene": "UniProtKB:H7C241",
  "gene_name": "Claudin-34",
  "term_id": "GO:0005923"
}